positive regulation of protein serine/threonine kinase activity [GO:0071902] (biological process) Relationships: is a type of GO:0045860; is a type of GO:0071900; positively regulates protein serine/threonine kinase activity [GO:0004674] Sources: GOC:mah Subtypes: GO:0043406, GO:0045737, positive regulation of protein kinase C activity [GO:1900020], positive regulation of cAMP-dependent protein kinase activity [GO:2000481] Definition: Any process that increases the rate, frequency, or extent of protein serine/threonine kinase activity.